carboxymethylhydantoinase activity [GO:0047771] (molecular function) Definition: Catalysis of the reaction: L-5-carboxymethylhydantoin + H2O = N-carbamoyl-L-aspartate + H+. Relationships: is a type of GO:0016812 Sources: EC:3.5.2.4, RHEA:12028 Also known as: L-5-carboxymethylhydantoin amidohydrolase activity, hydantoin hydrolase activity